{
  "gene": "UniProtKB:Q96IU2",
  "term_label": "positive regulation of canonical Wnt signaling pathway",
  "term_id": "GO:0090263",
  "gene_name": "Zinc finger BED domain-containing protein 3",
  "gene_symbol": "ZBED3"
}